paternal behavior [GO:0042712] (biological process) Relationships: is a type of parental behavior [GO:0060746] Sources: GOC:go_curators Definition: Male behaviors associated with the care and rearing offspring. Also known as: paternal behaviour